glutaminyl-peptide cyclotransferase activity [GO:0016603] (molecular function) Relationships: is a type of aminoacyltransferase activity [GO:0016755]; is a type of catalytic activity, acting on a protein [GO:0140096] Definition: Catalysis of the reaction: N-terminal L-glutaminyl-[peptide] = N-terminal 5-oxo-L-prolyl-[peptide] + NH4+. Sources: RHEA:23652 Also known as: glutaminyl-tRNA cyclotransferase activity, L-glutaminyl-peptide gamma-glutamyltransferase (cyclizing), glutaminyl cyclase activity, glutaminyl-transfer ribonucleate cyclotransferase activity